glucocorticoid secretion [GO:0035933] (biological process) Regulation: RO_0002211 by regulation of glucocorticoid secretion [GO:2000849]; negatively regulated by negative regulation of glucocorticoid secretion [GO:2000850]; positively regulated by positive regulation of glucocorticoid secretion [GO:2000851] Definition: The regulated release of any glucocorticoid hormone into the circulatory system. Glucocorticoids are a class of steroid hormones that regulate a variety of physiological processes, in particular control of the concentration of glucose in blood. Subtypes: corticosterone secretion [GO:0035934], cortisol secretion [GO:0043400] Relationships: is a type of GO:0035930 Sources: GOC:sl